positive regulation of rDNA heterochromatin formation [GO:2000749] (biological process) Relationships: is a type of GO:0031453; is a type of regulation of rDNA heterochromatin formation [GO:0061187]; positively regulates rDNA heterochromatin formation [GO:0000183] References: PMID:10899127 Definition: Any process that activates or increases the frequency, rate or extent of rDNA heterochromatin formation. Also known as: positive regulation of chromatin silencing at rDNA, positive regulation of chromatin silencing at ribosomal DNA, positive regulation of heterochromatic silencing at rDNA, positive regulation of rDNA chromatin silencing, positive regulation of rDNA heterochromatin assembly, positive regulation of ribosomal DNA heterochromatin assembly